positive regulation of cell cycle G1/S phase transition [GO:1902808] (BP) Relationships: is a type of positive regulation of cell cycle phase transition [GO:1901989]; is_a GO:1902806; positively regulates GO:0044843 Sources: GOC:TermGenie, GOC:mtg_cell_cycle, GO_REF:0000058 Definition: Any signaling pathway that activates or increases the activity of a cell cycle cyclin-dependent protein kinase to modulate the switch from G1 phase to S phase of the cell cycle. Also known as: up regulation of cell cycle G1/S phase transition, up-regulation of cell cycle G1/S phase transition, upregulation of cell cycle G1/S phase transition, activation of cell cycle G1/S phase transition Subtypes: positive regulation of G1/S transition of mitotic cell cycle [GO:1900087]